{
  "gene_name": "Vacuolar protein sorting-associated protein 28 homolog",
  "gene_symbol": "VPS28",
  "term_label": "protein-containing complex binding",
  "gene": "UniProtKB:Q9UK41",
  "term_id": "GO:0044877"
}